{
  "gene": "UniProtKB:Q9UKI9",
  "term_id": "GO:0000978",
  "gene_name": "POU domain, class 2, transcription factor 3",
  "term_label": "RNA polymerase II cis-regulatory region sequence-specific DNA binding",
  "gene_symbol": "POU2F3"
}